{
  "gene_name": "T-complex protein 11 X-linked protein 2",
  "term_id": "UNKNOWN:0001",
  "gene_symbol": "TCP11X2",
  "term_label": "Unknown molecular function",
  "gene": "UniProtKB:Q5H9J9"
}